{
  "gene_symbol": "INMT",
  "gene": "UniProtKB:O95050",
  "term_id": "GO:0008170",
  "term_label": "N-methyltransferase activity",
  "gene_name": "Indolethylamine N-methyltransferase"
}